{
  "gene_symbol": "INPP5E",
  "term_label": "nucleus",
  "gene": "UniProtKB:Q9NRR6",
  "term_id": "GO:0005634",
  "gene_name": "Phosphatidylinositol polyphosphate 5-phosphatase type IV"
}